{
  "term_id": "UNKNOWN:0001",
  "gene_name": "Glutaredoxin-related protein 5, mitochondrial",
  "term_label": "Unknown molecular function",
  "gene": "UniProtKB:Q86SX6",
  "gene_symbol": "GLRX5"
}